{
  "gene_symbol": "CTNNAL1",
  "term_id": "GO:0007266",
  "term_label": "Rho protein signal transduction",
  "gene": "UniProtKB:Q9UBT7",
  "gene_name": "Alpha-catulin"
}